{
  "term_label": "axon",
  "gene_symbol": "UNC80",
  "gene_name": "Protein unc-80 homolog",
  "term_id": "GO:0030424",
  "gene": "UniProtKB:Q8N2C7"
}